{
  "term_id": "UNKNOWN:0003",
  "gene_symbol": "COLQ",
  "gene": "UniProtKB:Q9Y215",
  "term_label": "Unknown cellular component",
  "gene_name": "Acetylcholinesterase collagenic tail peptide"
}